{
  "term_label": "cytoplasm",
  "gene_name": "Dynactin subunit 2",
  "gene": "UniProtKB:Q13561",
  "term_id": "GO:0005737",
  "gene_symbol": "DCTN2"
}